{
  "term_label": "cytosol",
  "gene_name": "Telomere length regulation protein TEL2 homolog",
  "gene_symbol": "TELO2",
  "gene": "UniProtKB:Q9Y4R8",
  "term_id": "GO:0005829"
}